{
  "term_label": "IPAF inflammasome complex",
  "gene_symbol": "NAIP",
  "gene_name": "Baculoviral IAP repeat-containing protein 1",
  "gene": "UniProtKB:Q13075",
  "term_id": "GO:0072557"
}